{
  "gene": "UniProtKB:P46063",
  "term_id": "GO:0000724",
  "gene_symbol": "RECQL",
  "term_label": "double-strand break repair via homologous recombination",
  "gene_name": "ATP-dependent DNA helicase Q1"
}